{
  "gene_name": "Tumor necrosis factor receptor superfamily member 11B",
  "term_label": "Unknown molecular function",
  "gene": "UniProtKB:O00300",
  "gene_symbol": "TNFRSF11B",
  "term_id": "UNKNOWN:0001"
}